4-hydroxy-tetrahydrodipicolinate synthase activity [GO:0008840] (molecular function) Relationships: is a type of hydro-lyase activity [GO:0016836] Definition: Catalysis of the reaction: pyruvate + L-aspartate-4-semialdehyde = (2S,4S)-4-hydroxy-2,3,4,5-tetrahydrodipicolinate + H2O. Also known as: dihydrodipicolinate synthase activity, DHDPS activity, L-aspartate-4-semialdehyde hydro-lyase (adding pyruvate and cyclizing), L-aspartate-4-semialdehyde hydro-lyase [adding pyruvate and cyclizing; (S)-2,3-dihydropyridine-2,6-dicarboxylate-forming], dihydrodipicolinate synthetase activity, dihydrodipicolinic acid synthase activity References: PMID:8993314 Sources: RHEA:34171